{
  "term_label": "positive regulation of innate immune response",
  "gene_symbol": "AKIRIN2",
  "gene": "UniProtKB:Q53H80",
  "term_id": "GO:0045089",
  "gene_name": "Akirin-2"
}